{
  "gene_symbol": "DEPP1",
  "gene": "UniProtKB:Q9NTK1",
  "term_id": "GO:0010506",
  "term_label": "regulation of autophagy",
  "gene_name": "Protein DEPP1"
}